{
  "term_id": "GO:0001764",
  "gene_name": "ABI gene family member 3",
  "gene_symbol": "ABI3",
  "gene": "UniProtKB:Q9P2A4",
  "term_label": "neuron migration"
}